{
  "gene_name": "CD177 antigen",
  "gene_symbol": "CD177",
  "gene": "UniProtKB:Q8N6Q3",
  "term_id": "GO:0044853",
  "term_label": "plasma membrane raft"
}